{
  "gene": "UniProtKB:Q9UFD9",
  "gene_symbol": "RIMBP3",
  "gene_name": "RIMS-binding protein 3A",
  "term_id": "GO:0007286",
  "term_label": "spermatid development"
}